single stranded viral RNA replication via double stranded DNA intermediate [GO:0039692] (biological process) Also known as: retroviral genome replication, viral ssRNA replication via dsDNA intermediate Regulation: regulated by regulation of single stranded viral RNA replication via double stranded DNA intermediate [GO:0045091]; negatively regulated by negative regulation of single stranded viral RNA replication via double stranded DNA intermediate [GO:0045869]; positively regulated by GO:0045870 Definition: A viral genome replication where the template is single-stranded RNA (ssRNA), and which proceeds via a double stranded DNA (dsDNA) intermediate molecule. Viral genomic RNA is first reverse transcribed into dsDNA, which integrates into the host chromosomal DNA, where it is transcribed by host RNA polymerase II. Relationships: is a type of viral RNA genome replication [GO:0039694]; has part reverse transcription [GO:0001171]; has part DNA-templated viral transcription [GO:0039695]; has part GO:0044826 Sources: GOC:bf, GOC:jl, ISBN:0198506732, VZ:1937